{
  "gene_name": "Fibroblast growth factor 14",
  "term_label": "cytoplasm",
  "gene": "UniProtKB:Q92915",
  "term_id": "GO:0005737",
  "gene_symbol": "FGF14"
}